{
  "term_id": "GO:0016477",
  "term_label": "cell migration",
  "gene": "UniProtKB:P16234",
  "gene_name": "Platelet-derived growth factor receptor alpha",
  "gene_symbol": "PDGFRA"
}